{
  "gene_name": "T cell receptor beta variable 4-1",
  "gene": "UniProtKB:A0A577",
  "term_id": "GO:0005886",
  "term_label": "plasma membrane",
  "gene_symbol": "TRBV4-1"
}